{
  "term_label": "centrosome",
  "term_id": "GO:0005813",
  "gene": "UniProtKB:Q496M5",
  "gene_name": "Inactive serine_threonine-protein kinase PLK5",
  "gene_symbol": "PLK5"
}